{
  "term_id": "GO:0007186",
  "gene": "UniProtKB:Q96LB1",
  "gene_symbol": "MRGPRX2",
  "gene_name": "Mas-related G-protein coupled receptor member X2",
  "term_label": "G protein-coupled receptor signaling pathway"
}